granzyme-mediated apoptotic signaling pathway [GO:0008626] (biological process) Also known as: apoptotic signaling pathway in response to granzyme, induction of apoptosis by granzyme Relationships: is a type of apoptotic signaling pathway [GO:0097190]; is a type of GO:0140507 References: PMID:17158907 Sources: GOC:mtg_apoptosis Definition: The series of molecular signals induced by granzymes which triggers the apoptotic death of a cell. The pathway starts with reception of a granzyme signal, and ends when the execution phase of apoptosis is triggered. Granzymes are serine proteases that are secreted by cytotoxic T cells and natural killer cells to induce apoptosis in target cells.